{
  "gene_symbol": "ALB",
  "gene": "UniProtKB:P02768",
  "term_id": "GO:0031667",
  "term_label": "response to nutrient levels",
  "gene_name": "Albumin"
}